{
  "term_id": "UNKNOWN:0002",
  "gene": "UniProtKB:A0A1B0GTR3",
  "gene_name": "Uncharacterized protein CXorf51A",
  "gene_symbol": "CXorf51A",
  "term_label": "Unknown biological process"
}